{
  "gene_name": "Uncharacterized protein",
  "gene_symbol": "A0A494C0B9",
  "gene": "UniProtKB:A0A494C0B9",
  "term_label": "Unknown cellular component",
  "term_id": "UNKNOWN:0003"
}